{
  "term_id": "GO:0007165",
  "gene_name": "Rho-related GTP-binding protein RhoV",
  "gene": "UniProtKB:Q96L33",
  "term_label": "signal transduction",
  "gene_symbol": "RHOV"
}